{
  "term_label": "tRNA pseudouridine synthesis",
  "term_id": "GO:0031119",
  "gene_name": "tRNA pseudouridine synthase-like 1",
  "gene_symbol": "PUSL1",
  "gene": "UniProtKB:Q8N0Z8"
}